{
  "term_label": "Unknown biological process",
  "gene_symbol": "PIK3CD-AS1",
  "gene_name": "Putative uncharacterized protein PIK3CD-AS1",
  "term_id": "UNKNOWN:0002",
  "gene": "UniProtKB:Q5SR53"
}